octanol catabolic process [GO:0046172] (biological process) Relationships: is a type of octanol metabolic process [GO:0006070]; is_a GO:0034310; is a type of GO:1903174 Sources: GOC:ai Also known as: octanol breakdown, octanol catabolism, octanol degradation Definition: The chemical reactions and pathways resulting in the breakdown of octanol, the 8-carbon alcohol with the formula C8H17OH.